{
  "term_id": "UNKNOWN:0001",
  "gene_symbol": "MIR1915HG",
  "gene_name": "Putative uncharacterized protein encoded by MIR1915-HG",
  "gene": "UniProtKB:Q5T4H9",
  "term_label": "Unknown molecular function"
}